walking behavior [GO:0090659] (biological process) Subtypes: adult walking behavior [GO:0007628], GO:0008346 Also known as: locomotor gait pattern Sources: GOC:tb Definition: The behavior of an organism relating to the progression of that organism along the ground by the process of lifting and setting down each leg. Relationships: is a type of locomotory behavior [GO:0007626]